{
  "term_id": "GO:0009313",
  "gene_name": "Sialidase-3",
  "gene_symbol": "NEU3",
  "gene": "UniProtKB:Q9UQ49",
  "term_label": "oligosaccharide catabolic process"
}